{
  "term_id": "GO:0015631",
  "gene_symbol": "TTLL9",
  "term_label": "tubulin binding",
  "gene_name": "Probable tubulin polyglutamylase TTLL9",
  "gene": "UniProtKB:Q3SXZ7"
}